{
  "gene_name": "17-beta-hydroxysteroid dehydrogenase 14",
  "term_label": "cytosol",
  "gene_symbol": "HSD17B14",
  "term_id": "GO:0005829",
  "gene": "UniProtKB:Q9BPX1"
}